biological regulation [GO:0065007] (biological process) Subtypes: regulation of pH [GO:0006885], regulation of buoyancy [GO:0031413], regulation of biological process [GO:0050789], regulation of brood size [GO:0060378], regulation of biological quality [GO:0065008], regulation of molecular function [GO:0065009], positive regulation of brood size [GO:0090727], negative regulation of brood size [GO:0090728], GO:0141191 Relationships: is a type of biological_process [GO:0008150] Also known as: regulation Sources: GOC:dph, GOC:isa_complete, GOC:mah, GOC:pr, GOC:vw Definition: Any process that modulates a measurable attribute of any biological process, quality or function.